{
  "term_label": "SRP-dependent cotranslational protein targeting to membrane, signal sequence recognition",
  "gene": "UniProtKB:P09132",
  "gene_name": "Signal recognition particle 19 kDa protein",
  "gene_symbol": "SRP19",
  "term_id": "GO:0006617"
}